accessory nerve development [GO:0021565] (biological process) Sources: GOC:cls, GOC:dgh, GOC:dph, GOC:jid, GO_REF:0000021 Also known as: cranial nerve XI development, spinal accessory nerve development, CN XI development, cranial nerve 11 development Relationships: is a type of cranial nerve development [GO:0021545] Definition: The process whose specific outcome is the progression of the accessory nerve over time, from its formation to the mature structure. In mice, the spinal branch of this motor nerve innervates the trapezius and the sternocleidomastoid muscles. The cranial branch joins the vagus nerve and innervates the same targets as the vagus nerve.